{
  "gene_symbol": "SAMHD1",
  "gene": "UniProtKB:Q9Y3Z3",
  "term_id": "GO:0005634",
  "gene_name": "Deoxynucleoside triphosphate triphosphohydrolase SAMHD1",
  "term_label": "nucleus"
}